{
  "gene_name": "Vacuolar protein sorting-associated protein 26A",
  "gene": "UniProtKB:O75436",
  "term_id": "GO:0042147",
  "term_label": "retrograde transport, endosome to Golgi",
  "gene_symbol": "VPS26A"
}